{
  "gene": "UniProtKB:Q8NCA9",
  "gene_symbol": "ZNF784",
  "term_label": "regulation of transcription by RNA polymerase II",
  "gene_name": "Zinc finger protein 784",
  "term_id": "GO:0006357"
}